{
  "term_label": "oxidoreductase activity",
  "gene": "UniProtKB:P47985",
  "gene_symbol": "UQCRFS1",
  "term_id": "GO:0016491",
  "gene_name": "Cytochrome b-c1 complex subunit Rieske, mitochondrial"
}